{
  "term_label": "HAUS complex",
  "gene_symbol": "HAUS3",
  "gene_name": "HAUS augmin-like complex subunit 3",
  "gene": "UniProtKB:Q68CZ6",
  "term_id": "GO:0070652"
}